{
  "term_label": "nucleus",
  "term_id": "GO:0005634",
  "gene": "UniProtKB:Q8IXZ3",
  "gene_name": "Transcription factor Sp8",
  "gene_symbol": "SP8"
}